1-alkenylglycerophosphoethanolamine O-acyltransferase activity [GO:0047166] (MF) Relationships: is a type of GO:0008374 Sources: EC:2.3.1.121, MetaCyc:2.3.1.121-RXN Also known as: acyl-CoA:1-alkenylglycerophosphoethanolamine O-acyltransferase activity Definition: Catalysis of the reaction: 1-alkenylglycerophosphoethanolamine + acyl-CoA = 1-alkenyl-2-acyl-glycerophosphoethanolamine + CoA.